{
  "gene": "UniProtKB:Q8WWH5",
  "term_label": "pseudouridine synthase activity",
  "gene_symbol": "TRUB1",
  "gene_name": "Pseudouridylate synthase TRUB1",
  "term_id": "GO:0009982"
}